negative regulation of nematode larval development, heterochronic [GO:0090446] (BP) References: PMID:17550772 Relationships: is a type of negative regulation of development, heterochronic [GO:0045961]; is a type of GO:0061064; is a type of regulation of nematode larval development, heterochronic [GO:0090444] Definition: Any process that modulates the consistent predetermined time point at which a nematode larva progresses from an initial condition to a later condition and decreases the rate at which this time point is reached.